{
  "gene_symbol": "TRBJ1-6",
  "gene": "UniProtKB:A0A0J9YWX3",
  "gene_name": "T cell receptor beta joining 1-6",
  "term_label": "Unknown cellular component",
  "term_id": "UNKNOWN:0003"
}